{
  "term_label": "phosphatidylserine binding",
  "gene_symbol": "HAVCR1",
  "gene_name": "Hepatitis A virus cellular receptor 1",
  "term_id": "GO:0001786",
  "gene": "UniProtKB:Q96D42"
}